{
  "gene_symbol": "FPR1",
  "term_id": "GO:0004982",
  "gene": "UniProtKB:P21462",
  "gene_name": "fMet-Leu-Phe receptor",
  "term_label": "N-formyl peptide receptor activity"
}